{
  "gene_symbol": "GOLPH3",
  "gene": "UniProtKB:Q9H4A6",
  "gene_name": "Golgi phosphoprotein 3",
  "term_label": "Golgi cisterna",
  "term_id": "GO:0031985"
}